{
  "term_label": "MOZ/MORF histone acetyltransferase complex",
  "gene": "UniProtKB:P55201",
  "gene_symbol": "BRPF1",
  "term_id": "GO:0070776",
  "gene_name": "Peregrin"
}